positive regulation of alkane biosynthetic process [GO:1901579] (biological process) Also known as: activation of alkane anabolism, activation of alkane biosynthesis, activation of alkane formation, activation of alkane synthesis, positive regulation of alkane anabolism, positive regulation of alkane biosynthesis, positive regulation of alkane formation, positive regulation of alkane synthesis, up regulation of alkane anabolism, up regulation of alkane biosynthesis, up regulation of alkane biosynthetic process, up regulation of alkane formation, up regulation of alkane synthesis, up-regulation of alkane anabolism, up-regulation of alkane biosynthesis, up-regulation of alkane biosynthetic process, up-regulation of alkane formation, up-regulation of alkane synthesis, upregulation of alkane anabolism, upregulation of alkane biosynthesis, upregulation of alkane biosynthetic process, upregulation of alkane formation, upregulation of alkane synthesis, activation of alkane biosynthetic process Sources: GOC:TermGenie Subtypes: positive regulation of methane biosynthetic process from dimethylamine [GO:1900320], positive regulation of methane biosynthetic process from trimethylamine [GO:1900332], positive regulation of methane biosynthetic process from 3-(methylthio)propionic acid [GO:1900335], GO:1900338, GO:1900341, positive regulation of methane biosynthetic process from dimethyl sulfide [GO:1900344], positive regulation of methane biosynthetic process from methanethiol [GO:1900347], GO:1900350, positive regulation of tridecane biosynthetic process [GO:1900886], GO:1900889, GO:1900898 Relationships: is a type of positive regulation of biosynthetic process [GO:0009891]; is a type of GO:1901577; positively regulates alkane biosynthetic process [GO:0043447] Definition: Any process that activates or increases the frequency, rate or extent of alkane biosynthetic process.